negative regulation of maltose transport [GO:1902344] (biological process) Definition: Any process that stops, prevents or reduces the frequency, rate or extent of maltose transport. Also known as: down regulation of maltose transport, down-regulation of maltose transport, downregulation of maltose transport, inhibition of maltose transport Relationships: is a type of negative regulation of transport [GO:0051051]; is a type of regulation of maltose transport [GO:1902343]; negatively regulates maltose transport [GO:0015768] References: PMID:23770568 Sources: GOC:TermGenie, GOC:dph